chromatin looping [GO:0140588] (biological process) Note: To describe the molecular function associated with chromatin looping, consider 'chromatin extrusion motor activity'; GO:0140584. Regulation: negatively regulated by GO:0160164 Relationships: is a type of chromatin organization [GO:0006325] Also known as: DNA looping, DNA loop extrusion, chromatin loop assembly, chromatin folding Definition: A chromatin organization process that starts with the loading of an extrusion motor (by an SMC family complex) onto the chromatin, followed by chromatin extrusion that stops at loop anchoring sites on the chromosome. References: PMID:32213323